diisopropyl-fluorophosphatase activity [GO:0047862] (molecular function) Relationships: is a type of hydrolase activity, acting on acid halide bonds [GO:0016824] Definition: Catalysis of the reaction: diisopropyl fluorophosphate + H2O = diisopropyl phosphate + fluoride + 2 H+. Sources: RHEA:24100 Also known as: DFPase activity, OPA anhydrase activity, OPAA activity, dialkylfluorophosphatase activity, diisopropyl phosphorofluoridate hydrolase activity, diisopropyl-fluorophosphate fluorohydrolase activity, diisopropylfluorophosphonate dehalogenase activity, diisopropylphosphofluoridase activity, isopropylphosphorofluoridase activity, organophosphate acid anhydrase activity, organophosphorus acid anhydrolase activity, somanase activity, tabunase activity